voltage-gated calcium channel activity involved in bundle of His cell action potential [GO:0086057] (molecular function) Relationships: is a type of voltage-gated calcium channel activity involved in cardiac muscle cell action potential [GO:0086007]; is part of membrane depolarization during bundle of His cell action potential [GO:0086048] Also known as: voltage-gated calcium channel activity involved in bundle of His cardiac muscle cell action potential Definition: Enables the transmembrane transfer of a calcium ion by a voltage-gated channel across the plasma membrane of a bundle of His cardiac muscle cell that contributes to the depolarization phase of an action potential. A voltage-gated channel is a channel whose open state is dependent on the voltage across the membrane in which it is embedded. Sources: GOC:BHF, GOC:mtg_cardiac_conduct_nov11